{
  "term_id": "GO:0007165",
  "gene": "UniProtKB:P24043",
  "term_label": "signal transduction",
  "gene_symbol": "LAMA2",
  "gene_name": "Laminin subunit alpha-2"
}